{
  "gene_symbol": "SIRT4",
  "gene_name": "NAD-dependent protein lipoamidase sirtuin-4, mitochondrial",
  "gene": "UniProtKB:Q9Y6E7",
  "term_id": "UNKNOWN:0002",
  "term_label": "Unknown biological process"
}